{
  "gene_symbol": "TBR1",
  "gene": "UniProtKB:Q16650",
  "term_id": "GO:0021902",
  "term_label": "commitment of neuronal cell to specific neuron type in forebrain",
  "gene_name": "T-box brain protein 1"
}